{
  "term_label": "carboxylesterase activity",
  "gene_name": "Cocaine esterase",
  "gene": "UniProtKB:O00748",
  "gene_symbol": "CES2",
  "term_id": "GO:0106435"
}